{
  "gene_symbol": "ATG9A",
  "gene": "UniProtKB:Q7Z3C6",
  "gene_name": "Autophagy-related protein 9A",
  "term_id": "GO:0000423",
  "term_label": "mitophagy"
}